RNA polymerase V core binding [GO:0001049] (molecular function) References: PMID:19110459 Sources: GOC:txnOH Definition: Binding to RNA polymerase V core enzyme, a multisubunit eukaryotic nuclear RNA polymerase found in plants and involved in production of noncoding transcripts at target loci for silencing. Relationships: is a type of RNA polymerase core enzyme binding [GO:0043175]